{
  "gene_name": "Keratin, type I cytoskeletal 9",
  "term_id": "GO:0030280",
  "term_label": "structural constituent of skin epidermis",
  "gene_symbol": "KRT9",
  "gene": "UniProtKB:P35527"
}